positive regulation of interleukin-34 production [GO:0150158] (biological process) Also known as: positive regulation of interleukin-34 biosynthetic process Sources: GOC:aruk Relationships: is a type of positive regulation of cytokine production [GO:0001819]; is a type of regulation of interleukin-34 production [GO:0150157]; positively regulates interleukin-34 production [GO:0150155] Definition: Any process that activates or increases the frequency, rate or extent of interleukin-34 production.